{
  "term_id": "GO:0005615",
  "term_label": "extracellular space",
  "gene": "UniProtKB:Q9UBX7",
  "gene_symbol": "KLK11",
  "gene_name": "Kallikrein-11"
}